{
  "term_label": "presynaptic active zone assembly",
  "gene_symbol": "PCDH17",
  "gene": "UniProtKB:O14917",
  "gene_name": "Protocadherin-17",
  "term_id": "GO:1904071"
}